{
  "term_label": "RNA polymerase II cis-regulatory region sequence-specific DNA binding",
  "term_id": "GO:0000978",
  "gene_symbol": "CPHXL2",
  "gene_name": "Cytoplasmic polyadenylated homeobox-like protein 2",
  "gene": "UniProtKB:A0A1W2PPK0"
}